cellular response to Thyroglobulin triiodothyronine [GO:1904017] (BP) Definition: Any process that results in a change in state or activity of a cell (in terms of movement, secretion, enzyme production, gene expression, etc.) as a result of a Thyroglobulin triiodothyronine stimulus. Relationships: is_a cellular response to chemical stimulus [GO:0070887]; is a type of response to Thyroglobulin triiodothyronine [GO:1904016] References: PMID:7531505 Sources: GOC:TermGenie, GO_REF:0000071